{
  "gene_name": "Protein HGH1 homolog",
  "gene_symbol": "HGH1",
  "gene": "UniProtKB:Q9BTY7",
  "term_id": "UNKNOWN:0001",
  "term_label": "Unknown molecular function"
}